{
  "term_id": "GO:0005852",
  "gene_name": "Eukaryotic translation initiation factor 3 subunit L",
  "term_label": "eukaryotic translation initiation factor 3 complex",
  "gene": "UniProtKB:Q9Y262",
  "gene_symbol": "EIF3L"
}